{
  "gene": "UniProtKB:P61160",
  "term_label": "Arp2/3 protein complex",
  "term_id": "GO:0005885",
  "gene_name": "Actin-related protein 2",
  "gene_symbol": "ACTR2"
}